{
  "term_label": "Unknown biological process",
  "gene": "UniProtKB:Q717R9",
  "gene_symbol": "CYS1",
  "gene_name": "Cystin-1",
  "term_id": "UNKNOWN:0002"
}